{
  "term_id": "GO:0005739",
  "gene": "UniProtKB:P10176",
  "gene_symbol": "COX8A",
  "term_label": "mitochondrion",
  "gene_name": "Cytochrome c oxidase subunit 8A, mitochondrial"
}